{
  "gene_symbol": "SF3A3",
  "gene_name": "Splicing factor 3A subunit 3",
  "term_label": "RNA binding",
  "gene": "UniProtKB:Q12874",
  "term_id": "GO:0003723"
}